{
  "term_id": "GO:0005634",
  "gene_name": "AT-rich interactive domain-containing protein 3B",
  "gene_symbol": "ARID3B",
  "term_label": "nucleus",
  "gene": "UniProtKB:Q8IVW6"
}